dinitrosyl-iron complex binding [GO:0035731] (molecular function) Relationships: is a type of metal cluster binding [GO:0051540] Also known as: DNDGIC binding, DNIC binding, dinitrosyl-diglutathionyl-iron complex binding Definition: Binding to a dinitrosyl-iron complex. Nitric oxide (NO) is stored as dinitrosyl-iron complexes, which form spontaneously from Glutathione (GSH), S-nitrosoglutathione, and trace amounts of ferrous ions, or by reaction of iron-sulfur centers with NO. References: PMID:10534443 Sources: GOC:BHF